{
  "term_label": "Unknown molecular function",
  "gene_symbol": "CENPVL1",
  "gene": "UniProtKB:A0A0U1RR11",
  "gene_name": "Centromere protein V-like protein 1",
  "term_id": "UNKNOWN:0001"
}